{
  "gene": "UniProtKB:Q14129",
  "gene_symbol": "DGCR6",
  "term_id": "UNKNOWN:0001",
  "term_label": "Unknown molecular function",
  "gene_name": "Protein DGCR6"
}